{
  "term_id": "GO:0070585",
  "term_label": "protein localization to mitochondrion",
  "gene": "UniProtKB:A0A2R8Y4M4",
  "gene_symbol": "LOC122513141",
  "gene_name": "RING-type domain-containing protein"
}